{
  "gene": "UniProtKB:Q8NEG0",
  "term_id": "UNKNOWN:0002",
  "gene_symbol": "GARIN6",
  "gene_name": "Golgi-associated RAB2 interactor protein 6",
  "term_label": "Unknown biological process"
}